{
  "term_id": "UNKNOWN:0001",
  "gene": "UniProtKB:A6NFA0",
  "term_label": "Unknown molecular function",
  "gene_name": "Protein SPATA31F3",
  "gene_symbol": "SPATA31F3"
}